positive regulation of elastin catabolic process [GO:0110015] (biological process) Definition: Any process that activates or increases the frequency, rate or extent of elastin catabolism, the chemical reactions and pathways resulting in the breakdown of elastin. Sources: GOC:BHF, GOC:BHF_miRNA, GOC:rph Relationships: is a type of positive regulation of protein catabolic process [GO:0045732]; is a type of regulation of elastin catabolic process [GO:0060310]; is a type of positive regulation of glycoprotein metabolic process [GO:1903020]; RO_0002213 elastin catabolic process [GO:0060309]